{
  "term_label": "stress fiber",
  "gene": "UniProtKB:Q9NR12",
  "gene_name": "PDZ and LIM domain protein 7",
  "gene_symbol": "PDLIM7",
  "term_id": "GO:0001725"
}